apical junction complex [GO:0043296] (cellular component) Definition: A functional unit located near the cell apex at the points of contact between epithelial cells, which in vertebrates is composed of the tight junction, the zonula adherens, and desmosomes and in some invertebrates, such as Drosophila, is composed of the subapical complex (SAC), the zonula adherens and the septate junction. Functions in the regulation of cell polarity, tissue integrity and intercellular adhesion and permeability. Also known as: apical cell junction complex, apical junction Relationships: is a type of GO:0005911 References: PMID:12525486, PMID:15196556 Sources: GOC:go_curators, GOC:kmv